CDP-diacylglycerol diphosphatase activity [GO:0008715] (molecular function) Also known as: CDP-diacylglycerol pyrophosphatase activity, CDP diacylglycerol hydrolase activity, CDP-diacylglycerol phosphatidylhydrolase activity, cytidine diphosphodiacylglycerol pyrophosphatase activity Relationships: is a type of pyrophosphatase activity [GO:0016462] Sources: EC:3.6.1.26, RHEA:15221 Definition: Catalysis of the reaction: CDP-diacylglycerol + H2O = a phosphatidate + CMP + 2 H+.